interleukin-33 receptor binding [GO:0002112] (molecular function) Definition: Binding to an interleukin-33 receptor. Also known as: IL-33, interleukin-33 receptor ligand Sources: GOC:hjd Relationships: is_a cytokine receptor binding [GO:0005126]